{
  "gene_name": "Cytochrome P450 2C8",
  "gene": "UniProtKB:P10632",
  "gene_symbol": "CYP2C8",
  "term_id": "GO:0016712",
  "term_label": "oxidoreductase activity, acting on paired donors, with incorporation or reduction of molecular oxygen, reduced flavin or flavoprotein as one donor, and incorporation of one atom of oxygen"
}